{
  "gene_name": "Kinesin-like protein KIF12",
  "term_id": "GO:0005871",
  "term_label": "kinesin complex",
  "gene_symbol": "KIF12",
  "gene": "UniProtKB:Q96FN5"
}